minus-end kinesin complex [GO:0005872] (CC) Relationships: is_a GO:0005871 Definition: Any complex that includes a dimer of molecules from the kinesin superfamily and any associated proteins, and moves towards the minus end of a microtubule. Sources: GOC:mah